regulation of chromatin organization [GO:1902275] (biological process) References: PMID:18314879 Sources: GOC:TermGenie, GOC:bf, GOC:vw, GO_REF:0000058 Relationships: is a type of GO:0051128; regulates GO:0006325 Definition: Any process that modulates the frequency, rate or extent of chromatin organization. Subtypes: regulation of heterochromatin formation [GO:0031445], GO:0120261, negative regulation of chromatin organization [GO:1905268], positive regulation of chromatin organization [GO:1905269] Also known as: regulation of chromatin organisation, regulation of establishment or maintenance of chromatin architecture, regulation of chromatin assembly or disassembly, regulation of chromatin assembly/disassembly, regulation of chromatin modification